{
  "gene_name": "Scaffold attachment factor B1",
  "term_id": "GO:0043565",
  "gene_symbol": "SAFB",
  "term_label": "sequence-specific DNA binding",
  "gene": "UniProtKB:Q15424"
}